{
  "term_label": "proteasome core complex, beta-subunit complex",
  "term_id": "GO:0019774",
  "gene": "UniProtKB:A5LHX3",
  "gene_symbol": "PSMB11",
  "gene_name": "Proteasome subunit beta type-11"
}